{
  "term_label": "positive regulation of feeding behavior",
  "gene_name": "Agouti-related protein",
  "term_id": "GO:2000253",
  "gene": "UniProtKB:O00253",
  "gene_symbol": "AGRP"
}